{
  "term_id": "GO:0031175",
  "term_label": "neuron projection development",
  "gene_name": "Receptor-type tyrosine-protein phosphatase zeta",
  "gene": "UniProtKB:P23471",
  "gene_symbol": "PTPRZ1"
}